4-methylaminobutyrate oxidase (demethylating) activity [GO:0102317] (molecular function) Definition: Catalysis of the reaction: 4-(methylamino)butyric acid + O2 + H2O = gamma-aminobutyric acid + formaldehyde + hydrogen peroxide. Relationships: is a type of oxidoreductase activity, acting on the CH-NH group of donors, oxygen as acceptor [GO:0016647] Sources: EC:1.5.3.19, GOC:pz